{
  "gene_name": "Copper transport protein ATOX1",
  "gene_symbol": "ATOX1",
  "gene": "UniProtKB:O00244",
  "term_label": "copper chaperone activity",
  "term_id": "GO:0016531"
}